NAD+ binding [GO:0070403] (molecular function) Definition: Binding to the oxidized form, NAD, of nicotinamide adenine dinucleotide, a coenzyme involved in many redox and biosynthetic reactions. Also known as: NAD (oxidized) binding, oxidized NAD binding, oxidized nicotinamide adenine dinucleotide binding, NAD binding Sources: GOC:mah Relationships: is a type of anion binding [GO:0043168]; is a type of NAD binding [GO:0051287]